{
  "term_id": "GO:0090385",
  "gene": "UniProtKB:Q9BZG1",
  "gene_name": "Ras-related protein Rab-34",
  "term_label": "phagosome-lysosome fusion",
  "gene_symbol": "RAB34"
}